{
  "term_id": "GO:0005737",
  "gene_symbol": "RNF13",
  "gene_name": "E3 ubiquitin-protein ligase RNF13",
  "term_label": "cytoplasm",
  "gene": "UniProtKB:O43567"
}